phosphatase complex [GO:1903293] (cellular component) Relationships: is a type of GO:1902494 Subtypes: protein serine/threonine phosphatase complex [GO:0008287], m7G(5')pppN diphosphatase complex [GO:0106095], protein tyrosine phosphatase complex [GO:1904096], acid phosphatase complex [GO:1904097], phosphatidylinositol phosphate phosphatase complex [GO:1904144] Note: An example of this is PTEN in human (P60484) in PMID:24766807 (inferred from direct assay). Definition: A protein complex which is capable of phosphatase activity. References: PMID:24766807 Sources: GOC:TermGenie, GOC:bhm, GO_REF:0000088